{
  "term_label": "RNA polymerase II cis-regulatory region sequence-specific DNA binding",
  "term_id": "GO:0000978",
  "gene_symbol": "ZNF490",
  "gene": "UniProtKB:Q9ULM2",
  "gene_name": "Zinc finger protein 490"
}